{
  "term_label": "cytosolic ribosome",
  "gene_symbol": "ISG15",
  "gene_name": "Ubiquitin-like protein ISG15",
  "gene": "UniProtKB:P05161",
  "term_id": "GO:0022626"
}